{
  "term_id": "GO:0031032",
  "gene": "UniProtKB:Q9Y2J2",
  "gene_name": "Band 4.1-like protein 3",
  "gene_symbol": "EPB41L3",
  "term_label": "actomyosin structure organization"
}